esterosome membrane [GO:0033118] (CC) References: PMID:2307702 Sources: GOC:ecd Definition: The lipid bilayer surrounding an esterosome. This membrane has characteristics of rough endoplasmic reticulum (RER) membranes. Relationships: is a type of cytoplasmic vesicle membrane [GO:0030659]; is a type of GO:0098588; is part of esterosome [GO:0033117]